{
  "term_id": "UNKNOWN:0001",
  "gene_name": "Proline-rich acidic protein 1",
  "gene_symbol": "PRAP1",
  "term_label": "Unknown molecular function",
  "gene": "UniProtKB:Q96NZ9"
}